{
  "term_label": "DNA-templated DNA replication",
  "gene_name": "ATPase WRNIP1",
  "gene_symbol": "WRNIP1",
  "gene": "UniProtKB:Q96S55",
  "term_id": "GO:0006261"
}